{
  "gene_name": "Serine_threonine-protein kinase 11-interacting protein",
  "term_id": "GO:0008104",
  "term_label": "intracellular protein localization",
  "gene_symbol": "STK11IP",
  "gene": "UniProtKB:Q8N1F8"
}